{
  "term_id": "GO:1990756",
  "gene_symbol": "PRAMEF8",
  "term_label": "ubiquitin-like ligase-substrate adaptor activity",
  "gene_name": "PRAME family member 8",
  "gene": "UniProtKB:Q5VWM4"
}